{
  "gene_name": "rRNA-processing protein FCF1 homolog",
  "term_id": "UNKNOWN:0001",
  "gene_symbol": "FCF1",
  "term_label": "Unknown molecular function",
  "gene": "UniProtKB:Q9Y324"
}